{
  "term_id": "GO:0033565",
  "gene_symbol": "STAM",
  "gene": "UniProtKB:Q92783",
  "term_label": "ESCRT-0 complex",
  "gene_name": "Signal transducing adapter molecule 1"
}